{
  "gene_name": "Cytochrome P450 4F3",
  "gene": "UniProtKB:Q08477",
  "term_id": "GO:0019369",
  "gene_symbol": "CYP4F3",
  "term_label": "arachidonate metabolic process"
}